{
  "term_label": "cytosol",
  "gene": "UniProtKB:Q96DE5",
  "gene_name": "Anaphase-promoting complex subunit 16",
  "term_id": "GO:0005829",
  "gene_symbol": "ANAPC16"
}